{
  "gene_symbol": "MT1H",
  "term_id": "GO:0006882",
  "gene_name": "Metallothionein-1H",
  "term_label": "intracellular zinc ion homeostasis",
  "gene": "UniProtKB:P80294"
}